{
  "gene": "UniProtKB:Q8TAE6",
  "term_id": "UNKNOWN:0002",
  "term_label": "Unknown biological process",
  "gene_symbol": "PPP1R14C",
  "gene_name": "Protein phosphatase 1 regulatory subunit 14C"
}